{
  "term_label": "regulation of transcription by RNA polymerase II",
  "gene_name": "Transcription factor SOX-5",
  "term_id": "GO:0006357",
  "gene_symbol": "SOX5",
  "gene": "UniProtKB:P35711"
}